{
  "gene_symbol": "SELENOK",
  "gene": "UniProtKB:Q9Y6D0",
  "term_id": "GO:0006816",
  "gene_name": "Selenoprotein K",
  "term_label": "calcium ion transport"
}